{
  "term_label": "plasma membrane",
  "gene_name": "Ras-related protein Ral-A",
  "gene": "UniProtKB:P11233",
  "term_id": "GO:0005886",
  "gene_symbol": "RALA"
}